{
  "gene_symbol": "DEFB105B",
  "term_label": "Unknown biological process",
  "gene": "UniProtKB:Q8NG35",
  "term_id": "UNKNOWN:0002",
  "gene_name": "Beta-defensin 105"
}